{
  "gene": "UniProtKB:Q8N428",
  "term_label": "polypeptide N-acetylgalactosaminyltransferase activity",
  "gene_name": "Polypeptide N-acetylgalactosaminyltransferase 16",
  "gene_symbol": "GALNT16",
  "term_id": "GO:0004653"
}